{
  "gene": "UniProtKB:Q70Z35",
  "term_label": "GTPase activator activity",
  "term_id": "GO:0005096",
  "gene_symbol": "PREX2",
  "gene_name": "Phosphatidylinositol 3,4,5-trisphosphate-dependent Rac exchanger 2 protein"
}